isoprene catabolic process [GO:0043613] (biological process) Definition: The chemical reactions and pathways resulting in the breakdown of isoprene, C5H8. Relationships: is a type of GO:0043611; is_a terpene catabolic process [GO:0046247]; is a type of GO:0120256 Also known as: 2-methyl-1,3-butadiene catabolic process, 2-methyl-1,3-butadiene catabolism, hemiterpene catabolic process, hemiterpene catabolism Sources: GOC:jl